{
  "gene_name": "Mitochondrial tRNA-specific 2-thiouridylase 1",
  "term_id": "GO:0002143",
  "gene": "UniProtKB:O75648",
  "gene_symbol": "TRMU",
  "term_label": "tRNA wobble position uridine thiolation"
}